progesterone 11-alpha-monooxygenase activity [GO:0050212] (molecular function) Sources: RHEA:18205 Also known as: progesterone 11a-monooxygenase activity, progesterone 11-alpha-hydroxylase activity, progesterone 11alpha-hydroxylase activity, progesterone 11alpha-monooxygenase activity, progesterone,hydrogen-donor:oxygen oxidoreductase (11alpha-hydroxylating) Definition: Catalysis of the reaction: AH2 + O2 + progesterone = 11alpha-hydroxyprogesterone + A + H2O. Relationships: is a type of GO:0050214